{
  "term_id": "GO:0042060",
  "gene": "UniProtKB:P15924",
  "gene_name": "Desmoplakin",
  "term_label": "wound healing",
  "gene_symbol": "DSP"
}